{
  "gene_name": "N-fatty-acyl-amino acid synthase_hydrolase PM20D1",
  "gene_symbol": "PM20D1",
  "gene": "UniProtKB:Q6GTS8",
  "term_label": "amide catabolic process",
  "term_id": "GO:0043605"
}